{
  "gene_symbol": "SPATA2",
  "term_id": "GO:0050727",
  "gene_name": "Spermatogenesis-associated protein 2",
  "term_label": "regulation of inflammatory response",
  "gene": "UniProtKB:Q9UM82"
}